{
  "term_id": "GO:0006955",
  "gene": "UniProtKB:O00590",
  "term_label": "immune response",
  "gene_symbol": "ACKR2",
  "gene_name": "Atypical chemokine receptor 2"
}